{
  "gene_name": "Formimidoyltransferase-cyclodeaminase",
  "term_label": "Unknown biological process",
  "gene": "UniProtKB:O95954",
  "term_id": "UNKNOWN:0002",
  "gene_symbol": "FTCD"
}